{
  "gene": "UniProtKB:P10636",
  "gene_name": "Microtubule-associated protein tau",
  "term_label": "neuron projection",
  "gene_symbol": "MAPT",
  "term_id": "GO:0043005"
}